biological phase [GO:0044848] (biological process) Definition: A distinct period or stage in a biological process or cycle. Note: Note that phases are is_a disjoint from other biological processes. happens_during relationships can operate between phases and other biological processes e.g. DNA replication happens_during S phase. Subtypes: GO:0022403, menstrual cycle phase [GO:0022601], hair cycle phase [GO:0044851], estrous cycle phase [GO:0060206], GO:0072690, anestrus phase [GO:0160266], GO:1990636 Sources: GOC:jl Relationships: is a type of GO:0008150